{
  "term_id": "GO:0042274",
  "gene_symbol": "RPS12",
  "term_label": "ribosomal small subunit biogenesis",
  "gene_name": "Small ribosomal subunit protein eS12",
  "gene": "UniProtKB:P25398"
}